{
  "term_label": "Unknown cellular component",
  "gene_symbol": "PPP1R37",
  "gene_name": "Protein phosphatase 1 regulatory subunit 37",
  "term_id": "UNKNOWN:0003",
  "gene": "UniProtKB:O75864"
}